{
  "gene_name": "Statherin",
  "gene": "UniProtKB:P02808",
  "term_id": "UNKNOWN:0001",
  "term_label": "Unknown molecular function",
  "gene_symbol": "STATH"
}